{
  "term_label": "Unknown cellular component",
  "gene": "UniProtKB:Q0VDD5",
  "term_id": "UNKNOWN:0003",
  "gene_name": "Putative uncharacterized protein encoded by MIR22HG",
  "gene_symbol": "MIR22HG"
}